{
  "gene_symbol": "SMO",
  "term_id": "GO:0007389",
  "term_label": "pattern specification process",
  "gene": "UniProtKB:Q99835",
  "gene_name": "Protein smoothened"
}